{
  "term_id": "GO:0001527",
  "term_label": "microfibril",
  "gene": "UniProtKB:P55001",
  "gene_symbol": "MFAP2",
  "gene_name": "Microfibrillar-associated protein 2"
}